{
  "term_id": "GO:0005737",
  "term_label": "cytoplasm",
  "gene": "UniProtKB:Q9BYX4",
  "gene_symbol": "IFIH1",
  "gene_name": "Interferon-induced helicase C domain-containing protein 1"
}